{
  "gene": "UniProtKB:Q16690",
  "gene_symbol": "DUSP5",
  "term_label": "nucleus",
  "gene_name": "Dual specificity protein phosphatase 5",
  "term_id": "GO:0005634"
}